{
  "term_id": "GO:0005778",
  "gene_symbol": "ABCD3",
  "term_label": "peroxisomal membrane",
  "gene": "UniProtKB:P28288",
  "gene_name": "ATP-binding cassette sub-family D member 3"
}